{
  "gene": "UniProtKB:Q32MZ4",
  "gene_symbol": "LRRFIP1",
  "term_label": "regulation of transcription by RNA polymerase II",
  "gene_name": "Leucine-rich repeat flightless-interacting protein 1",
  "term_id": "GO:0006357"
}